{
  "gene_name": "Sodium- and chloride-dependent glycine transporter 2",
  "term_label": "sodium ion transmembrane transport",
  "gene": "UniProtKB:Q9Y345",
  "term_id": "GO:0035725",
  "gene_symbol": "SLC6A5"
}